positive regulation of insulin secretion [GO:0032024] (biological process) Relationships: is a type of positive regulation of protein secretion [GO:0050714]; is a type of regulation of insulin secretion [GO:0050796]; is_a positive regulation of peptide hormone secretion [GO:0090277]; positively regulates insulin secretion [GO:0030073] Also known as: up regulation of insulin secretion, up-regulation of insulin secretion, upregulation of insulin secretion, activation of insulin secretion, stimulation of insulin secretion Sources: GOC:mah Definition: Any process that activates or increases the frequency, rate or extent of the regulated release of insulin. Subtypes: positive regulation of insulin secretion involved in cellular response to glucose stimulus [GO:0035774]